{
  "gene_name": "Chromodomain-helicase-DNA-binding protein 3",
  "gene_symbol": "CHD3",
  "gene": "UniProtKB:Q12873",
  "term_label": "chromatin binding",
  "term_id": "GO:0003682"
}